{
  "gene_name": "Receptor activity-modifying protein 3",
  "gene": "UniProtKB:O60896",
  "term_label": "coreceptor activity",
  "term_id": "GO:0015026",
  "gene_symbol": "RAMP3"
}